C-terminal protein methylation [GO:0006481] (biological process) Sources: GOC:ai Also known as: C-terminal protein amino acid methylation Relationships: is a type of GO:0006479; is a type of C-terminal protein amino acid modification [GO:0018410] Definition: The methylation of the C-terminal amino acid of a protein.